protein localization to bicellular tight junction [GO:1902396] (biological process) Relationships: is a type of protein localization to cell-cell junction [GO:0150105] Also known as: protein localisation in tight junction, protein localisation to tight junction, protein localization in tight junction References: PMID:18332111 Sources: GOC:TermGenie Definition: A process in which a protein is transported to, or maintained in, a location within a bicellular tight junction.